{
  "gene_name": "Peptide YY",
  "term_id": "GO:0005184",
  "gene": "UniProtKB:P10082",
  "gene_symbol": "PYY",
  "term_label": "neuropeptide hormone activity"
}